{
  "term_label": "cysteine-type endopeptidase inhibitor activity",
  "gene_name": "Cystatin-SN",
  "gene_symbol": "CST1",
  "term_id": "GO:0004869",
  "gene": "UniProtKB:P01037"
}